{
  "term_id": "UNKNOWN:0002",
  "gene_symbol": "HSPB3",
  "term_label": "Unknown biological process",
  "gene_name": "Heat shock protein beta-3",
  "gene": "UniProtKB:Q12988"
}